trichome branching [GO:0010091] (biological process) Definition: Any process involved in the formation of branches in plant hair cells. An example of this process is found in Arabidopsis thaliana. Sources: GOC:mtg_sensu, GOC:tair_curators Relationships: is a type of cell morphogenesis [GO:0000902]; is part of trichome morphogenesis [GO:0010090]